{
  "term_label": "Golgi to endosome transport",
  "gene": "UniProtKB:Q8N2H4",
  "term_id": "GO:0006895",
  "gene_name": "Protein SYS1 homolog",
  "gene_symbol": "SYS1"
}